regulation of T cell differentiation [GO:0045580] (biological process) Definition: Any process that modulates the frequency, rate or extent of T cell differentiation. Sources: GOC:go_curators Also known as: regulation of T lymphocyte differentiation, regulation of T-cell differentiation, regulation of T-lymphocyte differentiation, regulation of T cell development Note: Note that immunologists typically use the word 'development' to refer to cells of B or T cell lineages undergoing the process that GO describes as 'cell differentiation'. Relationships: is a type of GO:0045619; is a type of regulation of T cell activation [GO:0050863]; regulates GO:0030217 Subtypes: regulation of T cell differentiation in thymus [GO:0033081], GO:0033082, GO:0043380, negative regulation of T cell differentiation [GO:0045581], positive regulation of T cell differentiation [GO:0045582], regulation of cytotoxic T cell differentiation [GO:0045583], regulation of gamma-delta T cell differentiation [GO:0045586], regulation of regulatory T cell differentiation [GO:0045589], GO:0046637, GO:2000174